{
  "gene_name": "Probable ribonuclease 11",
  "gene": "UniProtKB:Q8TAA1",
  "gene_symbol": "RNASE11",
  "term_label": "defense response to Gram-positive bacterium",
  "term_id": "GO:0050830"
}